meiotic spindle assembly checkpoint signaling [GO:0033316] (biological process) Also known as: meiotic spindle assembly checkpoint, signal transduction involved in meiotic spindle assembly checkpoint Definition: A signal transduction process that contributes to a meiotic spindle assembly checkpoint, that delays the metaphase/anaphase transition of a meiotic cell cycle until the spindle is correctly assembled and chromosomes are attached to the spindle. Subtypes: meiosis I spindle assembly checkpoint signaling [GO:1905318] Relationships: is a type of meiotic spindle checkpoint signaling [GO:0044779]; is a type of spindle assembly checkpoint signaling [GO:0071173] Sources: GOC:mah